{
  "gene": "UniProtKB:Q6UWP8",
  "term_id": "UNKNOWN:0002",
  "gene_symbol": "SBSN",
  "term_label": "Unknown biological process",
  "gene_name": "Suprabasin"
}